{
  "gene_symbol": "TMEM59",
  "gene": "UniProtKB:Q9BXS4",
  "term_id": "GO:0005770",
  "gene_name": "Transmembrane protein 59",
  "term_label": "late endosome"
}